{
  "term_label": "nucleus",
  "gene_name": "Deoxyribonuclease-1",
  "gene_symbol": "DNASE1",
  "gene": "UniProtKB:P24855",
  "term_id": "GO:0005634"
}